microtubule binding [GO:0008017] (molecular function) Definition: Binding to a microtubule, a filament composed of tubulin monomers. Sources: GOC:krc Also known as: microtubule severing activity, microtubule/chromatin interaction Relationships: is a type of GO:0015631 Subtypes: microtubule plus-end binding [GO:0051010], microtubule minus-end binding [GO:0051011], microtubule lateral binding [GO:0099609]